response to pheromone regulating conjugation with mutual genetic exchange [GO:0000756] (biological process) Subtypes: adaptation to pheromone regulating conjugation with mutual genetic exchange [GO:0000760] Definition: Any process that results in a change in state or activity of a cell or an organism (in terms of movement, secretion, enzyme production, gene expression, etc.) as a result of a pheromone stimulus regulating the process of conjugation without cellular fusion. Also known as: response to pheromone triggering conjugation without cellular fusion Relationships: is a type of cell communication [GO:0007154]; is a type of cellular response to pheromone [GO:0071444]; regulates conjugation with mutual genetic exchange [GO:0000748] Sources: GOC:clt